{
  "gene_symbol": "GATA2",
  "term_label": "nucleus",
  "gene_name": "Endothelial transcription factor GATA-2",
  "term_id": "GO:0005634",
  "gene": "UniProtKB:P23769"
}